{
  "term_id": "GO:0000122",
  "gene_symbol": "WWP2",
  "term_label": "negative regulation of transcription by RNA polymerase II",
  "gene": "UniProtKB:O00308",
  "gene_name": "NEDD4-like E3 ubiquitin-protein ligase WWP2"
}